{
  "gene": "UniProtKB:Q8WY98",
  "gene_symbol": "TMEM234",
  "term_label": "Unknown biological process",
  "gene_name": "Transmembrane protein 234",
  "term_id": "UNKNOWN:0002"
}